centromere detachment from spindle pole body involved in meiotic chromosome organization [GO:0106212] (BP) Also known as: centromere detachment from SPB involved in meiotic chromosome organization, centromere detachment from spindle pole body involved in chromosome organization involved in meiotic cell cycle References: PMID:27611693 Sources: GOC:mah Relationships: is a type of chromosome organization involved in meiotic cell cycle [GO:0070192] Definition: The cell cycle process in which centromeres dissociate from the spindle pole body, contributing to the rearrangement of chromosomes into the orientation characteristic of meiotic prophase I.